{
  "gene_name": "OTU domain-containing protein 7B",
  "term_label": "K63-linked polyubiquitin modification-dependent protein binding",
  "term_id": "GO:0070530",
  "gene": "UniProtKB:Q6GQQ9",
  "gene_symbol": "OTUD7B"
}